{
  "term_id": "GO:0005634",
  "gene": "UniProtKB:Q8IZQ8",
  "gene_symbol": "MYOCD",
  "term_label": "nucleus",
  "gene_name": "Myocardin"
}